regulation of neuroinflammatory response [GO:0150077] (biological process) Definition: Any process that modulates the frequency, rate or extent of neuroinflammatory response. References: PMID:10981966, PMID:11099416, PMID:18164423 Sources: GOC:aruk, GOC:bc Relationships: is_a regulation of inflammatory response [GO:0050727]; regulates GO:0150076 Subtypes: positive regulation of neuroinflammatory response [GO:0150078], negative regulation of neuroinflammatory response [GO:0150079], regulation of microglial cell activation [GO:1903978]